{
  "gene_symbol": "CDK4",
  "term_label": "cyclin D1-CDK4 complex",
  "gene": "UniProtKB:P11802",
  "gene_name": "Cyclin-dependent kinase 4",
  "term_id": "GO:0097128"
}